{
  "gene_name": "S-methyl-5'-thioadenosine phosphorylase",
  "term_id": "GO:0017061",
  "term_label": "S-methyl-5-thioadenosine phosphorylase activity",
  "gene": "UniProtKB:Q13126",
  "gene_symbol": "MTAP"
}